{
  "gene_name": "EPM2A-interacting protein 1",
  "term_label": "Unknown cellular component",
  "gene": "UniProtKB:Q7L775",
  "term_id": "UNKNOWN:0003",
  "gene_symbol": "EPM2AIP1"
}